spliceosome-depend formation of circular RNA [GO:0160091] (biological process) Relationships: is a type of mRNA splicing, via spliceosome [GO:0000398] References: PMID:25768908, PMID:28625552 Definition: Formation of circular RNAs (circRNAs) by back-splicing circularization of pre-mRNAs in a spliceosome-dependent process.